{
  "gene_name": "Outer dense fiber protein 3-like protein 2",
  "gene_symbol": "ODF3L2",
  "term_id": "GO:0005856",
  "gene": "UniProtKB:Q3SX64",
  "term_label": "cytoskeleton"
}